{
  "term_label": "plasma membrane",
  "gene_name": "Sodium leak channel NALCN",
  "gene_symbol": "NALCN",
  "gene": "UniProtKB:Q8IZF0",
  "term_id": "GO:0005886"
}